{
  "gene_symbol": "MRGPRE",
  "term_label": "G protein-coupled receptor activity",
  "term_id": "GO:0004930",
  "gene_name": "Mas-related G-protein coupled receptor member E",
  "gene": "UniProtKB:Q86SM8"
}